{
  "gene_name": "Testicular haploid expressed gene protein",
  "term_id": "UNKNOWN:0003",
  "gene": "UniProtKB:Q9P2T0",
  "gene_symbol": "SPMAP2",
  "term_label": "Unknown cellular component"
}